{
  "gene_symbol": "ZNF732",
  "term_label": "regulation of DNA-templated transcription",
  "gene": "UniProtKB:B4DXR9",
  "gene_name": "Zinc finger protein 732",
  "term_id": "GO:0006355"
}